S-adenosyl-L-methionine transmembrane transport [GO:1901962] (biological process) Subtypes: mitochondrial S-adenosyl-L-methionine transmembrane transport [GO:1990543] Definition: The directed movement of S-adenosyl-L-methionine across a membrane. References: PMID:10497160 Sources: GOC:TermGenie Also known as: S-adenosylmethionine transmembrane transport, SAM transmembrane transport Relationships: is_a S-adenosyl-L-methionine transport [GO:0015805]; is a type of transmembrane transport [GO:0055085]